{
  "term_label": "nucleus",
  "term_id": "GO:0005634",
  "gene_name": "Homeobox protein engrailed-1",
  "gene_symbol": "EN1",
  "gene": "UniProtKB:Q05925"
}